{
  "term_id": "GO:0003697",
  "gene_symbol": "RAD51D",
  "gene_name": "DNA repair protein RAD51 homolog 4",
  "term_label": "single-stranded DNA binding",
  "gene": "UniProtKB:O75771"
}